pyrimidine ribonucleoside catabolic process [GO:0046133] (biological process) Sources: GOC:ai Also known as: pyrimidine ribonucleoside breakdown, pyrimidine ribonucleoside catabolism, pyrimidine ribonucleoside degradation Relationships: is a type of ribonucleoside catabolic process [GO:0042454]; is a type of pyrimidine ribonucleoside metabolic process [GO:0046131]; is a type of pyrimidine nucleoside catabolic process [GO:0046135] Definition: The chemical reactions and pathways resulting in the breakdown of any ribonucleoside, a nucleoside in which a pyrimidine base is linked to a ribose (beta-D-ribofuranose) molecule. Subtypes: GO:0006216, uridine catabolic process [GO:0006218]